{
  "term_label": "acetylcholine receptor binding",
  "term_id": "GO:0033130",
  "gene_symbol": "LY6S",
  "gene": "UniProtKB:P0DTL4",
  "gene_name": "Lymphocyte antigen 6S"
}